{
  "gene_symbol": "GPR152",
  "gene_name": "Probable G-protein coupled receptor 152",
  "term_label": "plasma membrane",
  "term_id": "GO:0005886",
  "gene": "UniProtKB:Q8TDT2"
}